{
  "term_label": "nucleosome array spacer activity",
  "gene": "UniProtKB:P51531",
  "gene_symbol": "SMARCA2",
  "term_id": "GO:0140750",
  "gene_name": "Probable global transcription activator SNF2L2"
}